{
  "gene_symbol": "PPP2CB",
  "gene": "UniProtKB:P62714",
  "gene_name": "Serine_threonine-protein phosphatase 2A catalytic subunit beta isoform",
  "term_label": "mitotic cell cycle",
  "term_id": "GO:0000278"
}